{
  "gene_name": "Latent-transforming growth factor beta-binding protein 1",
  "term_label": "Unknown biological process",
  "gene": "UniProtKB:Q14766",
  "term_id": "UNKNOWN:0002",
  "gene_symbol": "LTBP1"
}